{
  "gene_name": "Olfactory receptor 7C1",
  "gene": "UniProtKB:O76099",
  "term_id": "GO:0005886",
  "gene_symbol": "OR7C1",
  "term_label": "plasma membrane"
}